{
  "term_label": "cytoplasmic vesicle",
  "gene": "UniProtKB:Q66K66",
  "term_id": "GO:0031410",
  "gene_symbol": "TMEM198",
  "gene_name": "Transmembrane protein 198"
}